{
  "gene_name": "5-hydroxytryptamine receptor 3C",
  "term_id": "GO:0034220",
  "gene": "UniProtKB:Q8WXA8",
  "term_label": "monoatomic ion transmembrane transport",
  "gene_symbol": "HTR3C"
}